{
  "term_id": "GO:1902047",
  "gene_name": "Probable cation-transporting ATPase 13A5",
  "gene": "UniProtKB:Q4VNC0",
  "term_label": "polyamine transmembrane transport",
  "gene_symbol": "ATP13A5"
}